host symbiosome [GO:0043658] (cellular component) Subtypes: host bacteroid-containing symbiosome [GO:0043663] Definition: A double-enveloped cell compartment, composed of the endosymbiont with its plasmalemma (as inner envelope) and an outer envelope (the perisymbiontic membrane) derived from the host cell. Relationships: is a type of host intracellular membrane-bounded organelle [GO:0033648]; is a type of host cell cytoplasm part [GO:0033655] Sources: GOC:cc